{
  "gene_name": "NLR family CARD domain-containing protein 4",
  "term_id": "UNKNOWN:0001",
  "gene": "UniProtKB:Q9NPP4",
  "term_label": "Unknown molecular function",
  "gene_symbol": "NLRC4"
}